{
  "term_label": "nucleus",
  "term_id": "GO:0005634",
  "gene_name": "Alpha-globin transcription factor CP2",
  "gene": "UniProtKB:Q12800",
  "gene_symbol": "TFCP2"
}